corydaline synthase activity [GO:0050631] (molecular function) Also known as: S-adenosyl-L-methionine:protoberberine 13-C-methyltransferase activity Sources: EC:2.1.1.147, RHEA:14773 Definition: Catalysis of the reaction: S-adenosyl-L-methionine + 2 NADPH + palmatine = S-adenosyl-L-homocysteine + corydaline + 2 NADP+. Relationships: is a type of GO:0008168